{
  "term_id": "GO:0035102",
  "gene_name": "Polyhomeotic-like protein 1",
  "gene_symbol": "PHC1",
  "term_label": "PRC1 complex",
  "gene": "UniProtKB:P78364"
}